{
  "term_id": "GO:0051500",
  "gene_name": "D-aminoacyl-tRNA deacylase 2",
  "gene_symbol": "DTD2",
  "gene": "UniProtKB:Q96FN9",
  "term_label": "D-tyrosyl-tRNA(Tyr) deacylase activity"
}